{
  "gene": "UniProtKB:Q8NGN8",
  "term_id": "UNKNOWN:0002",
  "term_label": "Unknown biological process",
  "gene_symbol": "OR4A4P",
  "gene_name": "Putative olfactory receptor 4A4"
}